response to tetrachloromethane [GO:1904772] (biological process) Relationships: is a type of response to chemical [GO:0042221] Definition: Any process that results in a change in state or activity of a cell or an organism (in terms of movement, secretion, enzyme production, gene expression, etc.) as a result of a tetrachloromethane stimulus. References: PMID:7852267 Sources: GOC:TermGenie, GO_REF:0000071 Also known as: response to CCL4, response to carbon tetrachloride